dermal bone morphogenesis [GO:0061972] (BP) References: PMID:12588850, PMID:15003632 Definition: The process in which bone which forms superficially in the organism are generated and organized. Relationships: is a type of membrane bone morphogenesis [GO:0061973]